{
  "gene_symbol": "EVI2A",
  "gene": "UniProtKB:P22794",
  "gene_name": "Protein EVI2A",
  "term_label": "Unknown molecular function",
  "term_id": "UNKNOWN:0001"
}